{
  "gene_name": "Protein adenylyltransferase FICD",
  "term_label": "AMPylase activity",
  "gene_symbol": "FICD",
  "term_id": "GO:0070733",
  "gene": "UniProtKB:Q9BVA6"
}